rhizobactin 1021 biosynthetic process [GO:0019289] (biological process) Also known as: rhizobactin 1021 anabolism, rhizobactin 1021 biosynthesis, rhizobactin 1021 formation, rhizobactin 1021 synthesis, rhizobactin 1021 biosynthetic process, peptide formation, rhizobactin 1021 biosynthetic process, peptide modification Definition: The chemical reactions and pathways resulting in the formation of rhizobactin 1021, (E)-4-((3-(acetylhydroxyamino)propyl)-amino)-2-hydroxy-(2-(2-(3-(hydroxy(1-oxo-2-decenyl)amino)propyl)amino)-2-oxoethyl)-4-oxobutanoic acid, a siderophore produced by Sinorhizobium meliloti. Relationships: is a type of GO:0043604; is a type of carboxylic acid biosynthetic process [GO:0046394]; is a type of tertiary alcohol biosynthetic process [GO:1902645] References: PMID:11274118